mannotriose transport [GO:2001095] (biological process) Definition: The directed movement of a mannotrioseacetate into, out of or within a cell, or between cells, by means of some agent such as a transporter or pore. Relationships: is a type of trisaccharide transport [GO:2001088] Sources: GOC:mengo_curators Regulation: regulated by GO:1900327; negatively regulated by negative regulation of mannotriose transport [GO:1900328]; positively regulated by GO:1900329